{
  "gene": "UniProtKB:Q9C0D3",
  "term_id": "UNKNOWN:0001",
  "term_label": "Unknown molecular function",
  "gene_symbol": "ZYG11B",
  "gene_name": "Protein zyg-11 homolog B"
}